{
  "gene_name": "IQ domain-containing protein H",
  "gene": "UniProtKB:Q86VS3",
  "term_label": "Unknown molecular function",
  "gene_symbol": "IQCH",
  "term_id": "UNKNOWN:0001"
}